{
  "gene_symbol": "TNNI1",
  "term_id": "GO:0005861",
  "gene": "UniProtKB:P19237",
  "term_label": "troponin complex",
  "gene_name": "Troponin I, slow skeletal muscle"
}